cellular response to mechanical stimulus [GO:0071260] (biological process) Definition: Any process that results in a change in state or activity of a cell (in terms of movement, secretion, enzyme production, gene expression, etc.) as a result of a mechanical stimulus. Also known as: cellular mechanical stimulus response Sources: GOC:mah Relationships: is a type of response to mechanical stimulus [GO:0009612]; is a type of GO:0071214; is a type of cellular response to external stimulus [GO:0071496]